3-chlorocatechol biosynthetic process [GO:1901169] (biological process) Relationships: is a type of GO:0009713; is a type of benzene-containing compound metabolic process [GO:0042537]; is a type of organohalogen metabolic process [GO:0090345] Also known as: 3-chlorocatechol anabolism, 3-chlorocatechol biosynthesis, 3-chlorocatechol formation, 3-chlorocatechol synthesis Definition: The chemical reactions and pathways resulting in the formation of 3-chlorocatechol. Sources: GOC:TermGenie, GOC:yaf, UniPathway:UPA00083